{
  "term_label": "DNA-binding transcription factor activity, RNA polymerase II-specific",
  "gene_name": "Zinc finger protein 765",
  "term_id": "GO:0000981",
  "gene": "UniProtKB:Q7L2R6",
  "gene_symbol": "ZNF765"
}